{
  "gene": "UniProtKB:Q9H0D2",
  "term_id": "GO:0000118",
  "term_label": "histone deacetylase complex",
  "gene_name": "Zinc finger protein 541",
  "gene_symbol": "ZNF541"
}